{
  "term_id": "GO:0007623",
  "term_label": "circadian rhythm",
  "gene_symbol": "BMAL1",
  "gene_name": "Basic helix-loop-helix ARNT-like protein 1",
  "gene": "UniProtKB:O00327"
}